{
  "gene_name": "Protein phosphatase 1 regulatory subunit 3F",
  "term_id": "GO:2001069",
  "gene_symbol": "PPP1R3F",
  "gene": "UniProtKB:Q6ZSY5",
  "term_label": "glycogen binding"
}